bis(5'-adenosyl)-pentaphosphatase activity [GO:0034432] (molecular function) Definition: Catalysis of the reaction: P1-P6-bis(5'-adenosyl) pentaphosphate + H2O = AMP + adenosine 5'-tetraphosphate. References: PMID:10085096, PMID:9450008 Also known as: AP(5)A hydrolase activity, AP-5-A hydrolase activity, AP5A hydrolase activity, Ap5a pyrophosphohydrolase activity, diadenosine 5',5'''-P1,P6-pentaphosphate hydrolase activity Relationships: is a type of GO:0016462